{
  "term_id": "GO:0035082",
  "term_label": "axoneme assembly",
  "gene_symbol": "CPLANE2",
  "gene": "UniProtKB:Q9BU20",
  "gene_name": "Ciliogenesis and planar polarity effector 2"
}